positive regulation of T cell activation [GO:0050870] (biological process) Subtypes: T cell costimulation [GO:0031295], positive regulation of T cell proliferation [GO:0042102], positive regulation of T cell differentiation [GO:0045582], positive regulation of alpha-beta T cell activation [GO:0046635], positive regulation of gamma-delta T cell activation [GO:0046645], GO:1903905, positive regulation of T cell costimulation [GO:2000525], positive regulation of memory T cell activation [GO:2000568], positive regulation of T cell activation via T cell receptor contact with antigen bound to MHC molecule on antigen presenting cell [GO:2001190] Relationships: is a type of GO:0050863; is a type of GO:0051251; is_a positive regulation of leukocyte cell-cell adhesion [GO:1903039]; positively regulates GO:0042110 Definition: Any process that activates or increases the frequency, rate or extent of T cell activation. Sources: GOC:ai Also known as: positive regulation of T lymphocyte activation, positive regulation of T-cell activation, positive regulation of T-lymphocyte activation, up regulation of T cell activation, up-regulation of T cell activation, upregulation of T cell activation, activation of T cell activation, stimulation of T cell activation